regulation of syncytial blastoderm mitotic cell cycle [GO:0007348] (biological process) Sources: GOC:dph, GOC:go_curators, GOC:tb Relationships: is a type of regulation of mitotic cell cycle, embryonic [GO:0009794]; is a type of cell cycle process [GO:0022402]; regulates syncytial blastoderm mitotic cell cycle [GO:0035186] Subtypes: GO:0046003, positive regulation of syncytial blastoderm mitotic cell cycle [GO:0046004] Definition: A cell cycle process that modulates the rate or extent of the progression through the syncytial blastoderm mitotic cell cycle. Also known as: modulation of syncytial blastoderm cell cycle progression, regulation of progression through syncytial blastoderm mitotic cell cycle, regulation of syncytial blastoderm cell cycle, regulation of syncytial blastoderm cell cycle progression, syncytial blastoderm cell cycle modulation, syncytial blastoderm cell cycle regulation, syncytial blastoderm cell cycle regulator